{
  "term_id": "GO:1902969",
  "gene_symbol": "MCM6",
  "gene_name": "DNA replication licensing factor MCM6",
  "term_label": "mitotic DNA replication",
  "gene": "UniProtKB:Q14566"
}